{
  "term_label": "Unknown molecular function",
  "gene": "UniProtKB:B1AJZ9",
  "gene_symbol": "FHAD1",
  "gene_name": "Forkhead-associated domain-containing protein 1",
  "term_id": "UNKNOWN:0001"
}